{
  "gene_symbol": "ACTB",
  "gene": "UniProtKB:P60709",
  "term_id": "GO:0019901",
  "term_label": "protein kinase binding",
  "gene_name": "Actin, cytoplasmic 1"
}